high-affinity IgA receptor activity [GO:0002170] (molecular function) Definition: Combining with high affinity with an immunoglobulin of an IgA isotype via the Fc region, and transmitting the signal from one side of the membrane to the other to initiate a change in cell activity. Sources: GOC:hjd, GOC:signaling Also known as: high affinity IgA receptor activity Relationships: is a type of IgA receptor activity [GO:0019766]